oomycete sporangium development [GO:0075321] (biological process) Regulation: RO_0002211 by regulation of oomycete sporangium development [GO:0075322]; positively regulated by positive regulation of oomycete sporangium development [GO:0075323]; negatively regulated by GO:0075324 Sources: GOC:pamgo_curators Relationships: is a type of asexual sporulation [GO:0030436]; is a type of sporangium development [GO:0043582] Definition: The process that leads to the development of an oomycete sporangium, a single-celled or many-celled structure that germinates directly to form an infection hypha or differentiates, through specialized cleavage vesicles, into between 10 and 30 zoospores, which are laterally flagellated.